{
  "gene": "UniProtKB:Q8IX90",
  "gene_name": "Spindle and kinetochore-associated protein 3",
  "term_id": "GO:0000940",
  "term_label": "outer kinetochore",
  "gene_symbol": "SKA3"
}